negative regulation of pheromone-dependent signal transduction involved in conjugation with cellular fusion [GO:0090029] (biological process) Definition: Any process that decreases the frequency, rate or extent of pheromone-dependent signal transduction during conjugation with cellular fusion, a signal transduction process resulting in the relay, amplification or dampening of a signal generated in response to pheromone exposure in organisms that undergo conjugation with cellular fusion. Sources: GOC:dph, GOC:tb Relationships: is a type of regulation of pheromone-dependent signal transduction involved in conjugation with cellular fusion [GO:0010969]; is a type of GO:0060240; negatively regulates pheromone-dependent signal transduction involved in conjugation with cellular fusion [GO:0000750]